detection of stimulus involved in sensory perception [GO:0050906] (biological process) Definition: The series of events involved in sensory perception in which a sensory stimulus is received and converted into a molecular signal. Sources: GOC:ai, GOC:dos, GOC:dph Also known as: sensory detection of stimulus, sensory perception, sensory transduction of stimulus, sensory perception, stimulus detection, sensory transduction Relationships: is a type of detection of stimulus [GO:0051606]; is part of sensory perception [GO:0007600] Subtypes: GO:0050907, detection of temperature stimulus involved in sensory perception [GO:0050961], detection of light stimulus involved in sensory perception [GO:0050962], detection of electrical stimulus involved in sensory perception [GO:0050963], detection of mechanical stimulus involved in sensory perception [GO:0050974], detection of stimulus involved in sensory perception of pain [GO:0062149], detection of humidity stimulus involved in sensory perception [GO:0098512]